{
  "gene_name": "C-C chemokine receptor type 9",
  "term_id": "GO:0009897",
  "gene": "UniProtKB:P51686",
  "gene_symbol": "CCR9",
  "term_label": "external side of plasma membrane"
}